positive regulation of ATPase-coupled calcium transmembrane transporter activity [GO:1901896] (biological process) Definition: Any process that activates or increases the frequency, rate or extent of an ATPase-coupled calcium transmembrane transporter activity. Relationships: is a type of positive regulation of ion transmembrane transporter activity [GO:0032414]; is a type of GO:0032781; is a type of regulation of ATPase-coupled calcium transmembrane transporter activity [GO:1901894]; positively regulates GO:0005388 Also known as: activation of calcium pump, positive regulation of calcium pump, up regulation of calcium pump, up-regulation of calcium pump, upregulation of calcium pump, activation of ATP phosphohydrolase (Ca2+-transporting), activation of Ca(2+)-transporting ATPase activity, activation of Ca2+-pumping ATPase activity, activation of Ca2+-transporting ATPase activity, activation of calcium transporting ATPase activity, positive regulation of ATP phosphohydrolase (Ca2+-transporting), positive regulation of Ca(2+)-transporting ATPase activity, positive regulation of Ca2+-pumping ATPase activity, positive regulation of Ca2+-transporting ATPase activity, positive regulation of calcium transporting ATPase activity, positive regulation of calcium-transporting ATPase activity, up regulation of ATP phosphohydrolase (Ca2+-transporting), up regulation of Ca(2+)-transporting ATPase activity, up regulation of Ca2+-pumping ATPase activity, up regulation of Ca2+-transporting ATPase activity, up regulation of calcium transporting ATPase activity, up regulation of calcium-transporting ATPase activity, up-regulation of ATP phosphohydrolase (Ca2+-transporting), up-regulation of Ca(2+)-transporting ATPase activity, up-regulation of Ca2+-pumping ATPase activity, up-regulation of Ca2+-transporting ATPase activity, up-regulation of calcium transporting ATPase activity, up-regulation of calcium-transporting ATPase activity, upregulation of ATP phosphohydrolase (Ca2+-transporting), upregulation of Ca(2+)-transporting ATPase activity, upregulation of Ca2+-pumping ATPase activity, upregulation of Ca2+-transporting ATPase activity, upregulation of calcium transporting ATPase activity, upregulation of calcium-transporting ATPase activity, activation of calcium ABC transporter, activation of calcium efflux ATPase, activation of calcium-translocating P-type ATPase activity, activation of calcium-transporting ATPase activity, activation of plasma membrane Ca-ATPase, activation of sarco(endo)plasmic reticulum Ca2+-ATPase, activation of sarcoplasmic reticulum ATPase, positive regulation of calcium ABC transporter, positive regulation of calcium efflux ATPase, positive regulation of calcium-translocating P-type ATPase activity, positive regulation of plasma membrane Ca-ATPase, positive regulation of sarco(endo)plasmic reticulum Ca2+-ATPase, positive regulation of sarcoplasmic reticulum ATPase, up regulation of calcium ABC transporter, up regulation of calcium efflux ATPase, up regulation of calcium-translocating P-type ATPase activity, up regulation of plasma membrane Ca-ATPase, up regulation of sarco(endo)plasmic reticulum Ca2+-ATPase, up regulation of sarcoplasmic reticulum ATPase, up-regulation of calcium ABC transporter, up-regulation of calcium efflux ATPase, up-regulation of calcium-translocating P-type ATPase activity, up-regulation of plasma membrane Ca-ATPase, up-regulation of sarco(endo)plasmic reticulum Ca2+-ATPase, up-regulation of sarcoplasmic reticulum ATPase, upregulation of calcium ABC transporter, upregulation of calcium efflux ATPase, upregulation of calcium-translocating P-type ATPase activity, upregulation of plasma membrane Ca-ATPase, upregulation of sarco(endo)plasmic reticulum Ca2+-ATPase, upregulation of sarcoplasmic reticulum ATPase References: PMID:19708671 Sources: GOC:BHF, GOC:TermGenie, GOC:rl